{
  "term_label": "nucleus",
  "term_id": "GO:0005634",
  "gene_symbol": "CARF",
  "gene": "UniProtKB:Q8N187",
  "gene_name": "Calcium-responsive transcription factor"
}